{
  "term_id": "GO:0005886",
  "gene_name": "Putative vomeronasal receptor-like protein 4",
  "gene": "UniProtKB:Q8TDU5",
  "term_label": "plasma membrane",
  "gene_symbol": "VN1R17P"
}